{
  "gene_name": "Cyclic AMP-dependent transcription factor ATF-6 alpha",
  "term_label": "RNA polymerase II cis-regulatory region sequence-specific DNA binding",
  "gene": "UniProtKB:P18850",
  "term_id": "GO:0000978",
  "gene_symbol": "ATF6"
}